{
  "gene_symbol": "GRIN2A",
  "gene": "UniProtKB:Q12879",
  "gene_name": "Glutamate receptor ionotropic, NMDA 2A",
  "term_id": "GO:0060079",
  "term_label": "excitatory postsynaptic potential"
}